{
  "gene": "UniProtKB:Q8N782",
  "gene_name": "Zinc finger protein 525",
  "term_label": "regulation of DNA-templated transcription",
  "term_id": "GO:0006355",
  "gene_symbol": "ZNF525"
}